{
  "term_id": "GO:0012505",
  "gene_name": "E3 ubiquitin-protein ligase synoviolin",
  "term_label": "endomembrane system",
  "gene_symbol": "SYVN1",
  "gene": "UniProtKB:Q86TM6"
}